{
  "term_label": "kinocilium",
  "gene": "UniProtKB:A6NGW2",
  "gene_symbol": "STRCP1",
  "gene_name": "Putative stereocilin-like protein",
  "term_id": "GO:0060091"
}